medium-chain fatty-acyl-CoA metabolic process [GO:0036112] (biological process) Subtypes: medium-chain fatty-acyl-CoA catabolic process [GO:0036114] Also known as: medium-chain fatty acyl CoA metabolic process, medium-chain fatty acyl-CoA metabolism Definition: The chemical reactions and pathways involving medium-chain fatty-acyl-CoAs, any derivative of coenzyme A in which the sulfhydryl group is in a thioester linkage with a long-chain fatty-acyl group. A medium-chain fatty acid has an aliphatic tail containing 6 to 12 carbons. Note: While there is not universal consensus on the lengths of short-, medium-, long- and very-long-chain fatty acids, the GO uses the definitions in ChEBI (see CHEBI:26666, CHEBI:59554, CHEBI:15904 and CHEBI:27283). Relationships: is a type of fatty-acyl-CoA metabolic process [GO:0035337] Sources: GOC:pm